mitotic recombination [GO:0006312] (biological process) Sources: GOC:elh Relationships: is a type of DNA recombination [GO:0006310] Subtypes: telomere maintenance via recombination [GO:0000722], gene conversion at mating-type locus [GO:0007534] Regulation: regulated by regulation of mitotic recombination [GO:0000019]; negatively regulated by GO:0045950; positively regulated by positive regulation of mitotic recombination [GO:0045951] Definition: The exchange, reciprocal or nonreciprocal, of genetic material between one DNA molecule and a homologous DNA region that occurs during mitotic cell cycles.